defense response by callose deposition [GO:0052542] (biological process) Subtypes: defense response by callose deposition in cell wall [GO:0052544] Definition: Any process in which callose is transported to, and/or maintained in, a specific location during the defense response. Callose is a linear 1,3-beta-d-glucan formed from UDP-glucose and is found in certain plant cell walls. Regulation: regulated by regulation of defense response by callose deposition [GO:2000071] Also known as: callose deposition during defense response, callose localization during defense response Relationships: is a type of defense response [GO:0006952]; is a type of response to carbohydrate [GO:0009743]; is a type of callose localization [GO:0052545] Sources: GOC:mtg_pamgo_17jul06